negative regulation of interleukin-17A production [GO:0150152] (biological process) Relationships: is a type of negative regulation of interleukin-17 production [GO:0032700]; is a type of regulation of interleukin-17A production [GO:0150151]; negatively regulates interleukin-17A production [GO:0097087] Also known as: negative regulation of interleukin-17A biosynthetic process Definition: Any process that stops, prevents or reduces the frequency, rate or extent of interleukin-17A production. References: PMID:27901018 Sources: GOC:aruk